sulfoquinovosidase activity [GO:1990929] (molecular function) References: PMID:26878550 Sources: GOC:imk Relationships: is a type of GO:0016798 Definition: Catalyzes the hydrolysis of terminal non-reducing alpha-sulfoquinovoside residues in alpha-sulfoquinovosyl diacylglycerides and alpha-sulfoquinovosyl glycerol, generating alpha-sulfoquinovose.